{
  "gene_symbol": "GOLGA8S",
  "gene": "UniProtKB:H3BPF8",
  "gene_name": "Golgin subfamily A member 8S",
  "term_label": "Golgi cis cisterna",
  "term_id": "GO:0000137"
}